{
  "term_id": "GO:0015189",
  "gene_symbol": "SLC66A1LP",
  "gene_name": "Putative uncharacterized protein SLC66A1L",
  "gene": "UniProtKB:A1A4F0",
  "term_label": "L-lysine transmembrane transporter activity"
}